regulation of sarcomere organization [GO:0060297] (biological process) Also known as: regulation of sarcomere organisation Relationships: is a type of GO:0110020; is a type of regulation of supramolecular fiber organization [GO:1902903]; regulates sarcomere organization [GO:0045214] Sources: GOC:BHF, GOC:dph, GOC:tb Subtypes: positive regulation of sarcomere organization [GO:0060298], negative regulation of sarcomere organization [GO:0060299] Definition: Any process that modulates the rate, frequency or extent of myofibril assembly by organization of muscle actomyosin into sarcomeres. The sarcomere is the repeating unit of a myofibril in a muscle cell, composed of an array of overlapping thick and thin filaments between two adjacent Z discs.